{
  "gene_name": "Calcium homeostasis modulator protein 4",
  "gene": "UniProtKB:Q5JW98",
  "gene_symbol": "CALHM4",
  "term_label": "monoatomic cation channel activity",
  "term_id": "GO:0005261"
}